{
  "gene_symbol": "SPANXN2",
  "term_label": "Unknown cellular component",
  "gene_name": "Sperm protein associated with the nucleus on the X chromosome N2",
  "term_id": "UNKNOWN:0003",
  "gene": "UniProtKB:Q5MJ10"
}